{
  "term_id": "GO:0009913",
  "term_label": "epidermal cell differentiation",
  "gene_symbol": "OVOL3",
  "gene": "UniProtKB:O00110",
  "gene_name": "Putative transcription factor ovo-like protein 3"
}